{
  "gene_symbol": "MAPKAPK2",
  "gene_name": "MAP kinase-activated protein kinase 2",
  "term_label": "nucleus",
  "gene": "UniProtKB:P49137",
  "term_id": "GO:0005634"
}